L-lysine catabolic process using lysine 6-aminotransferase [GO:0033515] (biological process) Definition: The chemical reactions and pathways resulting in the breakdown of L-lysine into other compounds, including alpha-aminoadipate; in this pathway, L-lysine is converted to 2-aminoadipate-6-semialdehyde by lysine 6-aminotransferase. Sources: GOC:mah, MetaCyc:PWY-5298 Also known as: L-lysine breakdown using lysine 6-aminotransferase, L-lysine degradation using lysine 6-aminotransferase Relationships: is a type of GO:0019474